{
  "term_id": "GO:0000159",
  "gene_name": "Serine_threonine-protein phosphatase 2A regulatory subunit B'' subunit alpha",
  "term_label": "protein phosphatase type 2A complex",
  "gene": "UniProtKB:Q06190",
  "gene_symbol": "PPP2R3A"
}